{
  "gene_name": "Polymeric immunoglobulin receptor",
  "term_id": "GO:0002415",
  "gene_symbol": "PIGR",
  "term_label": "immunoglobulin transcytosis in epithelial cells mediated by polymeric immunoglobulin receptor",
  "gene": "UniProtKB:P01833"
}